histidyl-tRNA aminoacylation [GO:0006427] (biological process) Definition: The process of coupling histidine to histidyl-tRNA, catalyzed by histidyl-tRNA synthetase. The histidyl-tRNA synthetase is a class-II synthetase. The activated amino acid is transferred to the 3''-OH group of a histidine-accetping tRNA. Sources: GOC:mcc, ISBN:0716730510 Relationships: is a type of tRNA aminoacylation for protein translation [GO:0006418] Subtypes: mitochondrial histidyl-tRNA aminoacylation [GO:0070151]